{
  "gene_name": "Guanidinoacetate N-methyltransferase",
  "gene_symbol": "GAMT",
  "term_label": "creatine biosynthetic process",
  "gene": "UniProtKB:Q14353",
  "term_id": "GO:0006601"
}